Vma12-Vma22 assembly complex [GO:1990871] (CC) Definition: A protein complex that is involved in the assembly of the V-ATPase complex. In the budding yeast Saccharomyces cerevisiae, this complex consists of Vma12p and Vma22p. Relationships: is_a protein-containing complex [GO:0032991] References: PMID:9660861 Sources: GOC:rb